{
  "gene_name": "Zinc finger SWIM domain-containing protein 1",
  "gene": "UniProtKB:Q9BR11",
  "gene_symbol": "ZSWIM1",
  "term_id": "UNKNOWN:0003",
  "term_label": "Unknown cellular component"
}